melanin metabolic process [GO:0006582] (biological process) Subtypes: melanization defense response [GO:0035006], melanin biosynthetic process [GO:0042438], melanin catabolic process [GO:0046150] Sources: GOC:go_curators Also known as: melanin metabolism Relationships: is a type of phenol-containing compound metabolic process [GO:0018958]; is a type of secondary metabolic process [GO:0019748]; is a type of pigment metabolic process [GO:0042440] Definition: The chemical reactions and pathways involving melanins, pigments largely of animal origin. High molecular weight polymers of indole quinone, they are irregular polymeric structures and are divided into three groups: allomelanins in the plant kingdom and eumelanins and phaeomelanins in the animal kingdom.